bradykinin receptor activity [GO:0004947] (MF) Sources: GOC:ai Definition: Combining with bradykinin to initiate a change in cell activity. Relationships: is a type of G protein-coupled peptide receptor activity [GO:0008528]